{
  "term_label": "nucleus",
  "gene_symbol": "TSHZ1",
  "gene": "UniProtKB:Q6ZSZ6",
  "gene_name": "Teashirt homolog 1",
  "term_id": "GO:0005634"
}